{
  "term_id": "GO:0004197",
  "term_label": "cysteine-type endopeptidase activity",
  "gene": "UniProtKB:P29466",
  "gene_name": "Caspase-1",
  "gene_symbol": "CASP1"
}